{
  "term_id": "GO:0005886",
  "gene_name": "Beta-adducin",
  "gene": "UniProtKB:P35612",
  "gene_symbol": "ADD2",
  "term_label": "plasma membrane"
}